{
  "gene_name": "Protein FAM236D",
  "gene": "UniProtKB:A0A1B0GTK5",
  "gene_symbol": "FAM236D",
  "term_id": "UNKNOWN:0001",
  "term_label": "Unknown molecular function"
}